{
  "gene_symbol": "PYGM",
  "gene": "UniProtKB:P11217",
  "gene_name": "Glycogen phosphorylase, muscle form",
  "term_label": "glycogen phosphorylase activity",
  "term_id": "GO:0008184"
}